acid secretion [GO:0046717] (biological process) Sources: GOC:ai Subtypes: gastric acid secretion [GO:0001696], gamma-aminobutyric acid secretion [GO:0014051], bile acid secretion [GO:0032782], citric acid secretion [GO:0046720], formic acid secretion [GO:0046721], lactic acid secretion [GO:0046722], malic acid secretion [GO:0046723], oxalic acid secretion [GO:0046724] Definition: The controlled release of acid by a cell or a tissue. Relationships: is a type of secretion [GO:0046903]